{
  "gene": "UniProtKB:Q9NVA2",
  "term_id": "GO:0005940",
  "gene_symbol": "SEPTIN11",
  "term_label": "septin ring",
  "gene_name": "Septin-11"
}